{
  "gene_name": "Uncharacterized protein",
  "term_id": "UNKNOWN:0003",
  "term_label": "Unknown cellular component",
  "gene": "UniProtKB:A0A1W2PNU3",
  "gene_symbol": "LOC122455342"
}